{
  "gene": "UniProtKB:O96028",
  "term_label": "nucleus",
  "gene_name": "Histone-lysine N-methyltransferase NSD2",
  "gene_symbol": "NSD2",
  "term_id": "GO:0005634"
}